{
  "gene_name": "Ubiquitin-like modifier-activating enzyme 5",
  "gene_symbol": "UBA5",
  "term_label": "UFM1 activating enzyme activity",
  "term_id": "GO:0071566",
  "gene": "UniProtKB:Q9GZZ9"
}